{
  "gene_name": "Myelin P2 protein",
  "gene_symbol": "PMP2",
  "term_id": "GO:0005829",
  "gene": "UniProtKB:P02689",
  "term_label": "cytosol"
}